{
  "gene_name": "Advanced glycosylation end product-specific receptor",
  "term_id": "GO:1900272",
  "gene": "UniProtKB:Q15109",
  "term_label": "negative regulation of long-term synaptic potentiation",
  "gene_symbol": "AGER"
}